{
  "gene": "UniProtKB:Q5IJ48",
  "gene_name": "Protein crumbs homolog 2",
  "gene_symbol": "CRB2",
  "term_label": "heterophilic cell-cell adhesion",
  "term_id": "GO:0007157"
}